{
  "term_id": "UNKNOWN:0002",
  "gene_name": "NADH dehydrogenase [ubiquinone] 1 alpha subcomplex subunit 6",
  "gene_symbol": "NDUFA6",
  "term_label": "Unknown biological process",
  "gene": "UniProtKB:P56556"
}